{
  "gene": "UniProtKB:Q9UL19",
  "term_label": "N-acylphosphatidylethanolamine metabolic process",
  "term_id": "GO:0070292",
  "gene_name": "Phospholipase A and acyltransferase 4",
  "gene_symbol": "PLAAT4"
}